{
  "gene_name": "Protein SPO16 homolog",
  "term_label": "Unknown molecular function",
  "gene_symbol": "SPO16",
  "gene": "UniProtKB:Q5VVC0",
  "term_id": "UNKNOWN:0001"
}